{
  "term_label": "kinetochore binding",
  "gene_name": "Centromere protein H",
  "term_id": "GO:0043515",
  "gene_symbol": "CENPH",
  "gene": "UniProtKB:Q9H3R5"
}